protein alpha-1,2-demannosylation [GO:0036508] (biological process) Definition: The removal of one or more alpha 1,2-linked mannose residues from a mannosylated protein. Note: Consider also annotating to 'mannosyl-oligosaccharide 1,2-alpha-mannosidase activity ; GO:0004571'. References: PMID:21062743, PMID:25092655 Sources: GOC:PARL, GOC:bf Also known as: mannose trimming, glycoprotein mannose trimming Subtypes: endoplasmic reticulum mannose trimming [GO:1904380], mannose trimming involved in glycoprotein ERAD pathway [GO:1904382] Relationships: is a type of protein demannosylation [GO:0036507]; has part mannosyl-oligosaccharide 1,2-alpha-mannosidase activity [GO:0004571]